{
  "gene": "UniProtKB:O14771",
  "gene_name": "Zinc finger protein 213",
  "term_label": "RNA polymerase II cis-regulatory region sequence-specific DNA binding",
  "term_id": "GO:0000978",
  "gene_symbol": "ZNF213"
}